{
  "gene_symbol": "HACD1",
  "term_id": "GO:0030497",
  "term_label": "fatty acid elongation",
  "gene_name": "Very-long-chain (3R)-3-hydroxyacyl-CoA dehydratase 1",
  "gene": "UniProtKB:B0YJ81"
}